{
  "gene": "UniProtKB:Q99550",
  "term_id": "UNKNOWN:0001",
  "gene_name": "M-phase phosphoprotein 9",
  "term_label": "Unknown molecular function",
  "gene_symbol": "MPHOSPH9"
}